{
  "gene": "UniProtKB:Q96DI7",
  "term_id": "GO:0071013",
  "term_label": "catalytic step 2 spliceosome",
  "gene_name": "U5 small nuclear ribonucleoprotein 40 kDa protein",
  "gene_symbol": "SNRNP40"
}